anterior/posterior axon guidance [GO:0033564] (biological process) Definition: The process in which the migration of an axon growth cone is directed to a specific target site along the anterior-posterior body axis in response to a combination of attractive and repulsive cues. The anterior-posterior axis is defined by a line that runs from the head or mouth of an organism to the tail or opposite end of the organism. Sources: GOC:dph, GOC:kmv, GOC:tb Also known as: anterior-posterior axon guidance, anterior/posterior axon pathfinding Relationships: is a type of axon guidance [GO:0007411] Subtypes: GO:0097379, GO:0097380 Regulation: RO_0002211 by regulation of anterior/posterior axon guidance [GO:1905486]; negatively regulated by negative regulation of anterior/posterior axon guidance [GO:1905487]; positively regulated by GO:1905488